{
  "gene": "UniProtKB:O95177",
  "term_label": "Unknown cellular component",
  "gene_symbol": "GAS8-AS1",
  "gene_name": "Uncharacterized protein GAS8-AS1",
  "term_id": "UNKNOWN:0003"
}